{
  "term_id": "GO:0005634",
  "gene": "UniProtKB:Q6NX45",
  "gene_symbol": "ZNF774",
  "gene_name": "Zinc finger protein 774",
  "term_label": "nucleus"
}